negative regulation of receptor localization to synapse [GO:1902684] (biological process) References: PMID:22252129 Sources: GOC:TermGenie, GOC:kmv, GO_REF:0000058 Also known as: down regulation of receptor localisation to synapse, down regulation of receptor localization to synapse, down-regulation of receptor localisation to synapse, down-regulation of receptor localization to synapse, downregulation of receptor localisation to synapse, downregulation of receptor localization to synapse, negative regulation of receptor localisation to synapse, inhibition of receptor localisation to synapse, inhibition of receptor localization to synapse Relationships: is a type of negative regulation of biological process [GO:0048519]; is a type of regulation of receptor localization to synapse [GO:1902683]; negatively regulates receptor localization to synapse [GO:0097120] Definition: Any process that stops, prevents or reduces the frequency, rate or extent of receptor localization to synapse.